{
  "gene_symbol": "RFC2",
  "term_label": "DNA clamp loader activity",
  "gene_name": "Replication factor C subunit 2",
  "term_id": "GO:0003689",
  "gene": "UniProtKB:P35250"
}